{
  "term_id": "GO:0005615",
  "gene_name": "Neurturin",
  "gene_symbol": "NRTN",
  "term_label": "extracellular space",
  "gene": "UniProtKB:Q99748"
}